{
  "term_label": "ethanolaminephosphotransferase activity",
  "term_id": "GO:0004307",
  "gene_symbol": "CEPT1",
  "gene": "UniProtKB:Q9Y6K0",
  "gene_name": "Choline_ethanolaminephosphotransferase 1"
}